cyanate transport [GO:0015704] (BP) Definition: The directed movement of cyanate, NCO-, the anion of cyanic acid, into, out of or within a cell, or between cells, by means of some agent such as a transporter or pore. Relationships: is a type of one-carbon compound transport [GO:0019755]; is a type of nitrogen compound transport [GO:0071705] Sources: GOC:krc